{
  "gene_symbol": "IGKV1D-37",
  "gene_name": "Probable non-functional immunoglobulinn kappa variable 1D-37",
  "term_label": "Unknown molecular function",
  "gene": "UniProtKB:P0DSN7",
  "term_id": "UNKNOWN:0001"
}